{
  "gene_symbol": "ABCB10",
  "term_label": "Unknown biological process",
  "gene_name": "ATP-binding cassette sub-family B member 10, mitochondrial",
  "term_id": "UNKNOWN:0002",
  "gene": "UniProtKB:Q9NRK6"
}